{
  "gene_name": "Glycine amidinotransferase, mitochondrial",
  "term_label": "mitochondrial intermembrane space",
  "term_id": "GO:0005758",
  "gene": "UniProtKB:P50440",
  "gene_symbol": "GATM"
}